{
  "gene": "UniProtKB:P68032",
  "gene_symbol": "ACTC1",
  "term_label": "actin-myosin filament sliding",
  "gene_name": "Actin, alpha cardiac muscle 1",
  "term_id": "GO:0033275"
}